response to oxygen radical [GO:0000305] (biological process) Subtypes: GO:0000303, cellular response to oxygen radical [GO:0071450] Relationships: is a type of GO:0000302 Sources: GOC:krc, ISBN:0124325653 Definition: Any process that results in a change in state or activity of a cell or an organism (in terms of movement, secretion, enzyme production, gene expression, etc.) as a result of an oxygen radical stimulus. An oxygen radical is any oxygen species that carries a free electron; examples include hydroxyl radicals and the superoxide anion.